{
  "gene_symbol": "AURKA",
  "term_label": "nucleus",
  "gene_name": "Aurora kinase A",
  "gene": "UniProtKB:O14965",
  "term_id": "GO:0005634"
}